{
  "gene_symbol": "LINC01599",
  "gene": "UniProtKB:Q8WXQ3",
  "term_label": "Unknown cellular component",
  "gene_name": "Putative uncharacterized protein encoded by LINC01599",
  "term_id": "UNKNOWN:0003"
}